{
  "gene_name": "Proline-rich protein 20B",
  "term_label": "Unknown molecular function",
  "gene_symbol": "PRR20B",
  "term_id": "UNKNOWN:0001",
  "gene": "UniProtKB:P86481"
}